{
  "gene": "UniProtKB:P17677",
  "term_id": "GO:0016198",
  "gene_symbol": "GAP43",
  "term_label": "axon choice point recognition",
  "gene_name": "Neuromodulin"
}